negative regulation of ecdysteroid biosynthetic process [GO:0045997] (biological process) Relationships: is a type of regulation of ecdysteroid biosynthetic process [GO:0007554]; is a type of GO:0062014; is a type of GO:0090032; negatively regulates ecdysteroid biosynthetic process [GO:0045456] Definition: Any process that stops, prevents, or reduces the frequency, rate or extent of the chemical reactions and pathways resulting in the formation of ecdysteroids. Sources: GOC:go_curators Also known as: down regulation of ecdysteroid biosynthetic process, down-regulation of ecdysteroid biosynthetic process, downregulation of ecdysteroid biosynthetic process, negative regulation of ecdysteroid anabolism, negative regulation of ecdysteroid biosynthesis, negative regulation of ecdysteroid formation, negative regulation of ecdysteroid synthesis, inhibition of ecdysteroid biosynthetic process